{
  "term_id": "GO:0015141",
  "gene_name": "Mitochondrial dicarboxylate carrier",
  "term_label": "succinate transmembrane transporter activity",
  "gene": "UniProtKB:Q9UBX3",
  "gene_symbol": "SLC25A10"
}